high-affinity lysine transmembrane transporter activity [GO:0005292] (MF) Sources: GOC:mtg_transport Definition: Enables the transfer of lysine from one side of a membrane to the other. In high-affinity transport the transporter is able to bind the solute even if it is only present at very low concentrations. Also known as: high affinity lysine transporter activity, high affinity lysine transmembrane transporter activity Relationships: is a type of high-affinity basic amino acid transmembrane transporter activity [GO:0005287]; is a type of L-lysine transmembrane transporter activity [GO:0015189]